{
  "gene_name": "Pre-B-cell leukemia transcription factor 4",
  "gene_symbol": "PBX4",
  "gene": "UniProtKB:Q9BYU1",
  "term_id": "GO:0048568",
  "term_label": "embryonic organ development"
}